{
  "term_id": "GO:0043495",
  "gene_name": "Beclin 1-associated autophagy-related key regulator",
  "term_label": "protein-membrane adaptor activity",
  "gene": "UniProtKB:Q6ZNE5",
  "gene_symbol": "ATG14"
}